regulation of secondary shoot formation [GO:2000032] (biological process) Sources: GOC:obol Also known as: regulation of axillary shoot system formation, regulation of auxiliary shoot formation, regulation of axillary shoot formation, regulation of shoot branching Relationships: is a type of regulation of morphogenesis of a branching structure [GO:0060688]; is a type of regulation of plant organ formation [GO:1905428]; regulates GO:0010223 Definition: Any process that modulates the frequency, rate or extent of secondary shoot formation.